{
  "term_label": "Unknown biological process",
  "gene": "UniProtKB:P60369",
  "term_id": "UNKNOWN:0002",
  "gene_name": "Keratin-associated protein 10-3",
  "gene_symbol": "KRTAP10-3"
}